{
  "gene_symbol": "CRISP3",
  "gene": "UniProtKB:P54108",
  "term_id": "UNKNOWN:0002",
  "term_label": "Unknown biological process",
  "gene_name": "Cysteine-rich secretory protein 3"
}